cellular response to chondroitin 4'-sulfate [GO:1905442] (biological process) Relationships: is_a cellular response to nitrogen compound [GO:1901699]; is a type of GO:1901701; is a type of response to chondroitin 4'-sulfate [GO:1905441] Definition: Any process that results in a change in state or activity of a cell (in terms of movement, secretion, enzyme production, gene expression, etc.) as a result of a chondroitin 4'-sulfate stimulus. References: PMID:22365850 Sources: GOC:TermGenie, GO_REF:0000071